{
  "term_id": "GO:0017147",
  "gene_name": "Inactive tyrosine-protein kinase transmembrane receptor ROR1",
  "term_label": "Wnt-protein binding",
  "gene_symbol": "ROR1",
  "gene": "UniProtKB:Q01973"
}